{
  "term_label": "cell migration",
  "gene_name": "Cadherin-15",
  "term_id": "GO:0016477",
  "gene": "UniProtKB:P55291",
  "gene_symbol": "CDH15"
}